negative regulation of aecium development [GO:0075270] (biological process) Relationships: is_a negative regulation of spore-bearing organ development [GO:0075262]; is a type of regulation of aecium development [GO:0075268]; negatively regulates aecium development [GO:0075267] Sources: GOC:pamgo_curators Definition: Any process that stops, prevents, or reduces the frequency, rate or extent of aecium development, a process in which a cuplike structure containing chains of aeciospores is formed.